double fertilization forming two zygotes [GO:0009677] (BP) Definition: Rudimentary double fertilization where one of the two sperm nuclei from the pollen tube fuses with the egg nucleus to form a 2n zygote, and the other fuses with the ventral canal cell nucleus to form a second zygote, which soon degenerates. An example of this process is found in the Gnetophytes, such as Welwitschia mirabilis. Relationships: is a type of fertilization [GO:0009566] Sources: GOC:mtg_sensu, GOC:tb